{
  "gene": "UniProtKB:P31785",
  "gene_symbol": "IL2RG",
  "term_label": "external side of plasma membrane",
  "gene_name": "Cytokine receptor common subunit gamma",
  "term_id": "GO:0009897"
}